{
  "term_id": "GO:0005829",
  "gene_name": "E3 ubiquitin-protein ligase RNF8",
  "gene_symbol": "RNF8",
  "term_label": "cytosol",
  "gene": "UniProtKB:O76064"
}